protein import into peroxisome matrix, substrate release [GO:0044721] (biological process) Definition: The process by which the cargo protein is released into the peroxisomal matrix, following translocation across the membrane. References: PMID:21976670 Relationships: is a type of GO:0032984; is part of protein import into peroxisome matrix [GO:0016558]